{
  "term_id": "GO:0031209",
  "gene_symbol": "ABI2",
  "term_label": "SCAR complex",
  "gene": "UniProtKB:Q9NYB9",
  "gene_name": "Abl interactor 2"
}